{
  "gene_symbol": "TRAFD1",
  "term_label": "Unknown molecular function",
  "gene": "UniProtKB:O14545",
  "gene_name": "TRAF-type zinc finger domain-containing protein 1",
  "term_id": "UNKNOWN:0001"
}